{
  "term_id": "GO:0006123",
  "gene_symbol": "MT-CO3",
  "gene_name": "Cytochrome c oxidase subunit 3",
  "gene": "UniProtKB:P00414",
  "term_label": "mitochondrial electron transport, cytochrome c to oxygen"
}